{
  "term_label": "cellular response to heat",
  "gene_name": "Putative heat shock protein HSP 90-beta 2",
  "gene_symbol": "HSP90AB2P",
  "term_id": "GO:0034605",
  "gene": "UniProtKB:Q58FF8"
}